peripheral B cell positive selection [GO:0002350] (biological process) Definition: Any process leading to positive selection of B cells in the periphery. Positive selection is the process in which B or T cells are selected to survive based on signaling through their antigen receptors. Sources: GOC:jal Also known as: peripheral B lymphocyte positive selection, peripheral B-cell positive selection, peripheral B-lymphocyte positive selection Relationships: is a type of peripheral B cell selection [GO:0002343]; is a type of B cell positive selection [GO:0002346]